{
  "gene_name": "PGC-1 and ERR-induced regulator in muscle protein 1",
  "term_label": "response to muscle activity",
  "gene": "UniProtKB:Q5SV97",
  "term_id": "GO:0014850",
  "gene_symbol": "PERM1"
}